{
  "term_label": "long-term synaptic potentiation",
  "gene_name": "Glutamate receptor ionotropic, NMDA 2B",
  "gene": "UniProtKB:Q13224",
  "term_id": "GO:0060291",
  "gene_symbol": "GRIN2B"
}